{
  "gene": "UniProtKB:Q9UK32",
  "term_label": "TORC1 signaling",
  "gene_symbol": "RPS6KA6",
  "gene_name": "Ribosomal protein S6 kinase alpha-6",
  "term_id": "GO:0038202"
}